cytoskeletal motor activator activity [GO:0140660] (molecular function) Definition: Binds to and increases the activity of a motor protein. References: PMID:33221250 Also known as: motor activity activator activity Relationships: is a type of cytoskeletal motor regulator activity [GO:0140659]; is a type of molecular function activator activity [GO:0140677]; RO_0002213 GO:0003774